{
  "gene": "UniProtKB:Q76FK4",
  "gene_symbol": "NOL8",
  "gene_name": "Nucleolar protein 8",
  "term_id": "GO:0003723",
  "term_label": "RNA binding"
}